{
  "gene_name": "B melanoma antigen 2",
  "term_label": "Unknown cellular component",
  "gene": "UniProtKB:Q86Y30",
  "term_id": "UNKNOWN:0003",
  "gene_symbol": "BAGE2"
}